{
  "term_label": "membrane",
  "term_id": "GO:0016020",
  "gene_symbol": "OR10Z1",
  "gene_name": "Olfactory receptor 10Z1",
  "gene": "UniProtKB:Q8NGY1"
}